nuclear body [GO:0016604] (CC) Subtypes: nuclear dicing body [GO:0010445], PML body [GO:0016605], LYSP100-associated nuclear domain [GO:0016606], interchromatin granule [GO:0035061], sphere organelle [GO:0071601], cleavage body [GO:0071920], Gemini of Cajal bodies [GO:0097504], nuclear ribonucleoprotein granule [GO:0140168], nuclear exosome focus [GO:1990251] Relationships: is a type of GO:0043232; is part of nucleoplasm [GO:0005654] Definition: Membraneless organelle present in the nucleoplasm and usually visible by confocal microscopy. References: PMID:28577509